{
  "gene_name": "Late cornified envelope protein 3A",
  "gene_symbol": "LCE3A",
  "term_id": "UNKNOWN:0003",
  "term_label": "Unknown cellular component",
  "gene": "UniProtKB:Q5TA76"
}